G protein-coupled purinergic nucleotide receptor signaling pathway [GO:0035589] (biological process) References: PMID:9755289 Sources: GOC:BHF Relationships: is a type of purinergic nucleotide receptor signaling pathway [GO:0035590] Also known as: G-protein coupled purinergic nucleotide receptor signaling pathway, G-protein coupled purinergic nucleotide receptor signalling pathway, P2Y receptor signaling pathway Definition: A G protein-coupled receptor signaling pathway initiated by an extracellular purine nucleotide binding to its receptor, and ending with the regulation of a downstream cellular process.